{
  "term_id": "UNKNOWN:0003",
  "gene_name": "Keratin-associated protein 27-1",
  "gene": "UniProtKB:Q3LI81",
  "gene_symbol": "KRTAP27-1",
  "term_label": "Unknown cellular component"
}